phosphopantothenoylcysteine decarboxylase complex [GO:0071513] (CC) Note: See also the molecular function term 'acetolactate synthase activity ; GO:0003984'. Definition: A protein complex that catalyzes decarboxylation of 4'-phosphopantothenoylcysteine to yield 4'-phosphopantetheine; this is the third step in the biosynthesis of Coenzyme A. The complex is homotrimeric in many eukaryotes, but is a heterotrimer in Saccharomyces. References: PMID:19915539 Sources: GOC:jh Relationships: is a type of catalytic complex [GO:1902494]; is part of GO:0005737